{
  "gene": "UniProtKB:Q8IWE5",
  "gene_name": "Pleckstrin homology domain-containing family M member 2",
  "gene_symbol": "PLEKHM2",
  "term_id": "GO:0032880",
  "term_label": "regulation of protein localization"
}